trehalose synthase activity [GO:0102986] (molecular function) Definition: Catalysis of the reaction: an NDP-alpha-D-glucose + D-glucose = a ribonucleoside 5'-diphosphate + alpha,alpha-trehalose + H+. Relationships: is_a hexosyltransferase activity [GO:0016758] Sources: RHEA:47416 Note: Note that this term has a MetaCyc pathway reference as the pathway only has a single step.